{
  "term_label": "antigen processing and presentation of endogenous peptide antigen via MHC class Ib",
  "gene_symbol": "ULBP2",
  "gene_name": "UL16-binding protein 2",
  "term_id": "GO:0002476",
  "gene": "UniProtKB:Q9BZM5"
}